{
  "gene": "UniProtKB:P21583",
  "term_label": "positive regulation of melanocyte differentiation",
  "term_id": "GO:0045636",
  "gene_symbol": "KITLG",
  "gene_name": "Kit ligand"
}